{
  "gene_symbol": "MEP1A",
  "term_id": "GO:0140448",
  "term_label": "signaling receptor ligand precursor processing",
  "gene": "UniProtKB:Q16819",
  "gene_name": "Meprin A subunit alpha"
}